{
  "gene_name": "Cytokine receptor-like factor 1",
  "term_id": "GO:0004896",
  "gene_symbol": "CRLF1",
  "term_label": "cytokine receptor activity",
  "gene": "UniProtKB:O75462"
}